{
  "term_label": "positive regulation of transcription of nucleolar large rRNA by RNA polymerase I",
  "gene": "UniProtKB:Q13610",
  "term_id": "GO:1901838",
  "gene_name": "Periodic tryptophan protein 1 homolog",
  "gene_symbol": "PWP1"
}